{
  "gene_name": "Protein lin-7 homolog C",
  "term_id": "GO:0016323",
  "gene_symbol": "LIN7C",
  "term_label": "basolateral plasma membrane",
  "gene": "UniProtKB:Q9NUP9"
}